{
  "gene_name": "Zinc finger and BTB domain-containing protein 1",
  "gene_symbol": "ZBTB1",
  "gene": "UniProtKB:Q9Y2K1",
  "term_id": "GO:0001227",
  "term_label": "DNA-binding transcription repressor activity, RNA polymerase II-specific"
}